{
  "term_label": "nucleus",
  "gene_name": "Protein Mis18-alpha",
  "gene_symbol": "MIS18A",
  "term_id": "GO:0005634",
  "gene": "UniProtKB:Q9NYP9"
}